{
  "gene": "UniProtKB:P43699",
  "term_id": "GO:0006357",
  "term_label": "regulation of transcription by RNA polymerase II",
  "gene_name": "Homeobox protein Nkx-2.1",
  "gene_symbol": "NKX2-1"
}